{
  "gene_name": "Gamma-aminobutyric acid receptor subunit gamma-1",
  "gene_symbol": "GABRG1",
  "term_label": "synaptic transmission, GABAergic",
  "term_id": "GO:0051932",
  "gene": "UniProtKB:Q8N1C3"
}